{
  "gene": "UniProtKB:A0A1W2PR48",
  "gene_symbol": "TLE7",
  "gene_name": "Transducin-like enhancer protein 7",
  "term_id": "GO:0090090",
  "term_label": "negative regulation of canonical Wnt signaling pathway"
}